{
  "term_id": "GO:0005737",
  "term_label": "cytoplasm",
  "gene_symbol": "GRTP1",
  "gene_name": "Growth hormone-regulated TBC protein 1",
  "gene": "UniProtKB:Q5TC63"
}